{
  "gene_name": "Sperm flagellar protein 1",
  "gene": "UniProtKB:Q9Y4P9",
  "term_id": "GO:0051493",
  "term_label": "regulation of cytoskeleton organization",
  "gene_symbol": "SPEF1"
}